meiotic cytokinesis [GO:0033206] (biological process) Subtypes: meiosis I cytokinesis [GO:0007110], GO:0007111, male meiosis cytokinesis [GO:0007112], polar body extrusion after meiotic divisions [GO:0040038] Definition: A cell cycle process that results in the division of the cytoplasm of a cell after meiosis, resulting in the separation of the original cell into two daughter cells. Relationships: is a type of GO:0061640; is a type of GO:1903046 Sources: GOC:mtg_cell_cycle Also known as: cytokinesis after meiosis